glomerular capillary formation [GO:0072104] (biological process) Relationships: is a type of angiogenesis [GO:0001525]; is part of glomerulus vasculature morphogenesis [GO:0072103] Sources: GOC:mtg_kidney_jan10 Definition: The process that gives rise to a glomerular capillary. This process pertains to the initial formation of a structure from unspecified parts. Subtypes: mesonephric glomerular capillary formation [GO:0061249], metanephric glomerular capillary formation [GO:0072277]